{
  "term_label": "Unknown molecular function",
  "gene_symbol": "TSPAN15",
  "term_id": "UNKNOWN:0001",
  "gene_name": "Tetraspanin-15",
  "gene": "UniProtKB:O95858"
}